{
  "term_label": "caspase binding",
  "gene_name": "Nucleolar protein 3",
  "term_id": "GO:0089720",
  "gene": "UniProtKB:O60936",
  "gene_symbol": "NOL3"
}